{
  "term_id": "UNKNOWN:0001",
  "gene_name": "Pleckstrin homology-like domain family B member 2",
  "gene": "UniProtKB:Q86SQ0",
  "term_label": "Unknown molecular function",
  "gene_symbol": "PHLDB2"
}